regulation of mitochondrial DNA metabolic process [GO:1901858] (biological process) Also known as: regulation of mitochondrial DNA metabolism, regulation of mtDNA metabolic process, regulation of mtDNA metabolism Definition: Any process that modulates the frequency, rate or extent of mitochondrial DNA metabolic process. References: PMID:23150719 Sources: GOC:TermGenie, GOC:yaf Subtypes: regulation of mitochondrial DNA replication [GO:0090296], negative regulation of mitochondrial DNA metabolic process [GO:1901859], positive regulation of mitochondrial DNA metabolic process [GO:1901860] Relationships: is a type of regulation of DNA metabolic process [GO:0051052]; regulates mitochondrial DNA metabolic process [GO:0032042]